{
  "gene_name": "Interferon beta",
  "term_id": "GO:0060337",
  "gene": "UniProtKB:P01574",
  "term_label": "type I interferon-mediated signaling pathway",
  "gene_symbol": "IFNB1"
}